protein deglycation, glyoxal removal [GO:0036529] (biological process) References: PMID:25416785 Sources: GOC:PARL, GOC:bf Relationships: is a type of protein deglycation [GO:0036525]; is a type of glycolate biosynthetic process [GO:0046295]; is a type of glyoxal metabolic process [GO:1903189] Also known as: protein deglycation of glyoxal-glycated protein Definition: The removal of glyoxal from a glycated protein, to form glycolate and a deglycated protein.